regulation of conidiophore stalk development [GO:0070799] (BP) Relationships: is a type of regulation of developmental process [GO:0050793]; is a type of regulation of reproductive process [GO:2000241]; regulates conidiophore stalk development [GO:0070788] Definition: Any process that modulates the frequency, rate or extent of conidiophore stalk development, a process that leads to the formation of a conidiophore stalk. The conidiophore stalk is part of a specialized hypha that extends aerially from the growth substrate and supports structures from which conidia, or asexual spores, develop. Subtypes: negative regulation of conidiophore stalk development [GO:0070800], positive regulation of conidiophore stalk development [GO:0070801] Sources: GOC:mah